N-acetyl-beta-D-glucosaminide beta-(1,3)-galactosyltransferase activity [GO:0008499] (molecular function) References: PMID:10212226 Sources: RHEA:53432 Also known as: beta-1,3-GalTase activity, beta3Gal-Ts activity, UDP-Gal:beta-GlcNAc beta-1,3-galactosyltransferase activity, UDP-galactose beta-N-acetylglucosamine beta-1,3-galactosyltransferase activity, UDP-galactose:beta-N-acetylglucosamine beta-1,3-galactosyltransferase activity Relationships: is_a UDP-galactosyltransferase activity [GO:0035250]; is a type of GO:0048531 Definition: Catalysis of the reaction: an N-acetyl-beta-D-glucosaminyl derivative + UDP-alpha-D-galactose = a beta-D-galactosyl-(1->3)-N-acetyl-beta-D-glucosaminyl derivative + H+ + UDP.